negative regulation of oxytocin production [GO:0140669] (biological process) Definition: Any process that stops, prevents, or reduces the rate of production of oxytocin. Relationships: is_a negative regulation of gene expression [GO:0010629]; is a type of regulation of oxytocin production [GO:0140667]; negatively regulates oxytocin production [GO:0036162] References: PMID:25096581